tryptophan dimethylallyltransferase activity [GO:0050364] (molecular function) Also known as: 4-(gamma,gamma-dimethylallyl)tryptophan synthase activity, DMAT synthetase activity, dimethylallyl-diphosphate:L-tryptophan dimethylallyltransferase activity, dimethylallylpyrophosphate:L-tryptophan dimethylallyltransferase activity, dimethylallylpyrophosphate:tryptophan dimethylallyl transferase activity, dimethylallyltryptophan synthetase activity Relationships: is a type of transferase activity, transferring alkyl or aryl (other than methyl) groups [GO:0016765] Definition: Catalysis of the reaction: dimethylallyl diphosphate + L-tryptophan = diphosphate + 4-(3-methylbut-2-enyl)-L-tryptophan. Sources: EC:2.5.1.34, MetaCyc:TRYPTOPHAN-DIMETHYLALLYLTRANSFERASE-RXN